{
  "term_label": "cysteine-type endopeptidase activity",
  "term_id": "GO:0004197",
  "gene_symbol": "CTSS",
  "gene": "UniProtKB:P25774",
  "gene_name": "Cathepsin S"
}